{
  "gene": "UniProtKB:Q9HBW0",
  "term_id": "GO:0005737",
  "gene_symbol": "LPAR2",
  "gene_name": "Lysophosphatidic acid receptor 2",
  "term_label": "cytoplasm"
}